{
  "gene": "UniProtKB:P27816",
  "term_label": "microtubule binding",
  "term_id": "GO:0008017",
  "gene_symbol": "MAP4",
  "gene_name": "Microtubule-associated protein 4"
}